garland nephrocyte differentiation [GO:0061321] (biological process) Also known as: garland cell differentiation Relationships: is a type of nephrocyte differentiation [GO:0061319]; is part of embryonic development via the syncytial blastoderm [GO:0001700] Definition: The process in which a relatively unspecialized cell acquires the specialized structural and/or functional features of a garland nephrocyte. A garland nephrocyte is an insect renal cell that filters hemolymph and forms a ring with other garland nephrocytes around the esophagus. Differentiation includes the processes involved in commitment of a cell to a specific fate and its subsequent development to the mature state. References: PMID:19783135 Sources: CL:0000486, GOC:dph, GOC:mtg_kidney_jan10, GOC:sart